{
  "gene_name": "Mitochondrial ribonuclease P catalytic subunit",
  "term_label": "mitochondrial ribonuclease P complex",
  "gene_symbol": "PRORP",
  "term_id": "GO:0030678",
  "gene": "UniProtKB:O15091"
}